{
  "term_label": "actin cytoskeleton",
  "term_id": "GO:0015629",
  "gene_name": "Actin-binding LIM protein 1",
  "gene": "UniProtKB:O14639",
  "gene_symbol": "ABLIM1"
}